{
  "gene_name": "Putative uncharacterized protein LOC645739",
  "gene": "UniProtKB:Q9H521",
  "gene_symbol": "Q9H521",
  "term_label": "Unknown biological process",
  "term_id": "UNKNOWN:0002"
}